{
  "term_label": "inositol-1,4,5-trisphosphate 5-phosphatase activity",
  "gene_name": "Synaptojanin-2",
  "gene": "UniProtKB:O15056",
  "gene_symbol": "SYNJ2",
  "term_id": "GO:0052658"
}